{
  "gene_symbol": "WASHC1",
  "term_id": "UNKNOWN:0001",
  "term_label": "Unknown molecular function",
  "gene": "UniProtKB:A8K0Z3",
  "gene_name": "WASH complex subunit 1"
}